{
  "gene_symbol": "PCDHGA4",
  "gene_name": "Protocadherin gamma-A4",
  "gene": "UniProtKB:Q9Y5G9",
  "term_label": "cell adhesion molecule binding",
  "term_id": "GO:0050839"
}